negative regulation of dehydroaustinol biosynthetic process [GO:1900650] (biological process) Definition: Any process that stops, prevents or reduces the frequency, rate or extent of dehydroaustinol biosynthetic process. Sources: GOC:TermGenie, GOC:di Also known as: down regulation of dehydroaustinol anabolism, down regulation of dehydroaustinol biosynthesis, down regulation of dehydroaustinol biosynthetic process, down regulation of dehydroaustinol formation, down regulation of dehydroaustinol synthesis, down-regulation of dehydroaustinol anabolism, down-regulation of dehydroaustinol biosynthesis, down-regulation of dehydroaustinol biosynthetic process, down-regulation of dehydroaustinol formation, down-regulation of dehydroaustinol synthesis, downregulation of dehydroaustinol anabolism, downregulation of dehydroaustinol biosynthesis, downregulation of dehydroaustinol biosynthetic process, downregulation of dehydroaustinol formation, downregulation of dehydroaustinol synthesis, inhibition of dehydroaustinol anabolism, inhibition of dehydroaustinol biosynthesis, inhibition of dehydroaustinol formation, inhibition of dehydroaustinol synthesis, negative regulation of dehydroaustinol anabolism, negative regulation of dehydroaustinol biosynthesis, negative regulation of dehydroaustinol formation, negative regulation of dehydroaustinol synthesis, inhibition of dehydroaustinol biosynthetic process Relationships: is a type of negative regulation of secondary metabolite biosynthetic process [GO:1900377]; is a type of regulation of dehydroaustinol biosynthetic process [GO:1900649]; negatively regulates dehydroaustinol biosynthetic process [GO:1900563]